antigen processing and presentation of endogenous antigen [GO:0019883] (biological process) Relationships: is a type of antigen processing and presentation [GO:0019882] Also known as: antigen presentation, endogenous antigen Subtypes: antigen processing and presentation of endogenous peptide antigen [GO:0002483], GO:0048006 References: PMID:15771591, PMID:15928678 Sources: GOC:add, ISBN:0781735149 Definition: The process in which an antigen-presenting cell expresses antigen (peptide or lipid) of endogenous origin on its cell surface in association with an MHC protein complex.